{
  "gene_name": "Methyltransferase-like protein 25B",
  "gene_symbol": "METTL25B",
  "term_id": "UNKNOWN:0003",
  "term_label": "Unknown cellular component",
  "gene": "UniProtKB:Q96FB5"
}